{
  "term_label": "chloride transmembrane transport",
  "gene_name": "Gamma-aminobutyric acid receptor subunit pi",
  "gene_symbol": "GABRP",
  "gene": "UniProtKB:O00591",
  "term_id": "GO:1902476"
}